thrombospondin receptor activity [GO:0070053] (MF) Relationships: is a type of GO:0038023 Sources: GOC:BHF, GOC:signaling, GOC:vk Definition: Combining with thrombospondin and transmitting the signal to initiate a change in cell activity.